prostate gland morphogenesis [GO:0060512] (biological process) Relationships: is a type of GO:0003006; is a type of GO:0022612; is part of GO:0030850 References: PMID:18977204 Sources: GOC:dph Definition: The process in which the anatomical structures of a prostate gland are generated and organized.